{
  "term_id": "GO:0006260",
  "gene_symbol": "RPA3",
  "term_label": "DNA replication",
  "gene": "UniProtKB:P35244",
  "gene_name": "Replication protein A 14 kDa subunit"
}